establishment of apical/basal cell polarity [GO:0035089] (biological process) Definition: The specification and formation of the polarity of a cell along its apical/basal axis. Sources: GOC:bf Relationships: is a type of GO:0035088; is a type of establishment of monopolar cell polarity [GO:0061162] Subtypes: establishment of epithelial cell apical/basal polarity [GO:0045198]